{
  "gene_name": "Microtubule-associated protein RP_EB family member 3",
  "gene": "UniProtKB:Q9UPY8",
  "term_label": "spindle assembly",
  "gene_symbol": "MAPRE3",
  "term_id": "GO:0051225"
}